{
  "term_label": "cell-cell adhesion",
  "gene_name": "Integrin beta-like protein 1",
  "term_id": "GO:0098609",
  "gene_symbol": "ITGBL1",
  "gene": "UniProtKB:O95965"
}